{
  "term_label": "immune response",
  "gene": "UniProtKB:P25311",
  "term_id": "GO:0006955",
  "gene_name": "Zinc-alpha-2-glycoprotein",
  "gene_symbol": "AZGP1"
}